{
  "term_label": "sodium ion transmembrane transport",
  "gene": "UniProtKB:P31645",
  "gene_name": "Sodium-dependent serotonin transporter",
  "term_id": "GO:0035725",
  "gene_symbol": "SLC6A4"
}